{
  "term_id": "GO:0048488",
  "gene": "UniProtKB:Q2LD37",
  "term_label": "synaptic vesicle endocytosis",
  "gene_name": "Bridge-like lipid transfer protein family member 1",
  "gene_symbol": "BLTP1"
}